proline:proton symporter activity [GO:0005297] (molecular function) Relationships: is a type of GO:0005280; is a type of carboxylic acid transmembrane transporter activity [GO:0046943] Definition: Enables the transfer of a solute or solutes from one side of a membrane to the other according to the reaction: proline(out) + H+(out) = proline(in) + H+(in). Also known as: hydrogen/proline transporter Sources: GOC:ai